{
  "term_label": "nucleus",
  "gene_name": "Transcription factor Spi-C",
  "gene": "UniProtKB:Q8N5J4",
  "term_id": "GO:0005634",
  "gene_symbol": "SPIC"
}